{
  "gene_symbol": "DSP",
  "gene": "UniProtKB:P15924",
  "term_label": "intermediate filament",
  "gene_name": "Desmoplakin",
  "term_id": "GO:0005882"
}